positive regulation of cyclin-dependent protein kinase activity [GO:1904031] (BP) Also known as: up regulation of cyclin-dependent protein kinase activity, up-regulation of cyclin-dependent protein kinase activity, upregulation of cyclin-dependent protein kinase activity, activation of cyclin-dependent protein kinase activity Relationships: is a type of GO:0045860; RO_0002213 cyclin-dependent protein kinase activity [GO:0097472] References: PMID:22995177 Sources: GOC:TermGenie, GOC:als, GO_REF:0000059 Subtypes: positive regulation of cyclin-dependent protein serine/threonine kinase activity [GO:0045737] Definition: Any process that activates or increases the frequency, rate or extent of cyclin-dependent protein kinase activity.